{
  "gene": "UniProtKB:Q96IZ6",
  "term_id": "UNKNOWN:0003",
  "gene_name": "tRNA N(3)-methylcytidine methyltransferase METTL2A",
  "term_label": "Unknown cellular component",
  "gene_symbol": "METTL2A"
}